glucagon secretion [GO:0070091] (biological process) Relationships: is a type of peptide hormone secretion [GO:0030072] Definition: The regulated release of glucagon from secretory granules in the A (alpha) cells of the pancreas (islets of Langerhans). Sources: GOC:BHF, GOC:rl Regulation: regulated by regulation of glucagon secretion [GO:0070092]; negatively regulated by GO:0070093; positively regulated by positive regulation of glucagon secretion [GO:0070094]